{
  "gene_name": "Glutamate receptor ionotropic, kainate 4",
  "term_id": "GO:0032983",
  "gene_symbol": "GRIK4",
  "gene": "UniProtKB:Q16099",
  "term_label": "kainate selective glutamate receptor complex"
}